{
  "term_label": "myosin II complex",
  "gene_symbol": "MYH15",
  "gene_name": "Myosin-15",
  "gene": "UniProtKB:Q9Y2K3",
  "term_id": "GO:0016460"
}